{
  "term_label": "plasma membrane",
  "gene": "UniProtKB:O94844",
  "gene_name": "Rho-related BTB domain-containing protein 1",
  "term_id": "GO:0005886",
  "gene_symbol": "RHOBTB1"
}